{
  "gene_name": "Histone acetyltransferase KAT2B",
  "term_id": "GO:0006338",
  "gene_symbol": "KAT2B",
  "term_label": "chromatin remodeling",
  "gene": "UniProtKB:Q92831"
}